membrane depolarization during bundle of His cell action potential [GO:0086048] (biological process) Also known as: membrane depolarization during bundle of His cardiac muscle cell action potential Definition: The process in which bundle of His cardiac muscle cell membrane potential changes in the depolarizing direction from the negative resting potential towards the positive membrane potential that will be the peak of the action potential. Sources: GOC:BHF, GOC:mtg_cardiac_conduct_nov11 Relationships: is a type of membrane depolarization during cardiac muscle cell action potential [GO:0086012]; is part of bundle of His cell action potential [GO:0086043]